{
  "gene": "UniProtKB:Q9UGJ0",
  "gene_symbol": "PRKAG2",
  "term_label": "nucleus",
  "gene_name": "5'-AMP-activated protein kinase subunit gamma-2",
  "term_id": "GO:0005634"
}